Golgi apparatus N-glycan mannose trimming [GO:1904381] (BP) References: PMID:10915796, PMID:30858582, PMID:35536965 Also known as: mannose trimming in Golgi, Golgi apparatus mannose trimming, mannose trimming in Golgi apparatus, protein alpha-1,2-demannosylation in Golgi apparatus, protein alpha-1,2-demannosylation in Golgi complex, mannose trimming in cis-Golgi, protein alpha-1,2-demannosylation in Golgi ribbon, glycoprotein mannose trimming in Golgi apparatus, glycoprotein mannose trimming in Golgi complex, glycoprotein mannose trimming in Golgi ribbon Relationships: is a type of N-glycan processing [GO:0006491] Definition: The trimming, in the Golgi apparatus, of the protein newly attached high-mannose-type N-glycans by mannosidases to produce paucimannose-type N-glycans.